{
  "gene": "UniProtKB:A8MTW9",
  "gene_name": "Putative uncharacterized protein ENSP00000380674",
  "term_id": "UNKNOWN:0001",
  "gene_symbol": "A8MTW9",
  "term_label": "Unknown molecular function"
}